{
  "gene_name": "Neurofilament light polypeptide",
  "gene_symbol": "NEFL",
  "gene": "UniProtKB:P07196",
  "term_id": "GO:0030424",
  "term_label": "axon"
}